glutamine family amino acid biosynthetic process [GO:0009084] (biological process) Relationships: is a type of glutamine family amino acid metabolic process [GO:0009064]; is a type of L-amino acid biosynthetic process [GO:0170034]; is a type of GO:0170038 Definition: The chemical reactions and pathways resulting in the formation of amino acids of the glutamine family, comprising arginine, glutamate, glutamine and proline. Also known as: glutamine family amino acid anabolism, glutamine family amino acid biosynthesis, glutamine family amino acid formation, glutamine family amino acid synthesis Subtypes: L-arginine biosynthetic process [GO:0006526], glutamate biosynthetic process [GO:0006537], glutamine biosynthetic process [GO:0006542], L-proline biosynthetic process [GO:0055129] Sources: GOC:ai